{
  "gene_symbol": "P2RY14",
  "gene": "UniProtKB:Q15391",
  "term_label": "Unknown cellular component",
  "term_id": "UNKNOWN:0003",
  "gene_name": "P2Y purinoceptor 14"
}